type-I dockerin domain binding [GO:1990308] (MF) Relationships: is a type of protein domain specific binding [GO:0019904] Definition: Binding to a type-I dockerin domain of a protein. Type-I dockerin domain is the binding partner of type-1 cohesin domain. References: PMID:23195689, PMID:24080387 Sources: GOC:mengo_curators